{
  "gene_name": "Proenkephalin-B",
  "term_label": "plasma membrane",
  "term_id": "GO:0005886",
  "gene_symbol": "PDYN",
  "gene": "UniProtKB:P01213"
}